{
  "gene": "UniProtKB:A0A5B9",
  "term_id": "GO:0042105",
  "gene_symbol": "TRBC2",
  "term_label": "alpha-beta T cell receptor complex",
  "gene_name": "T cell receptor beta constant 2"
}